regulation of adenine biosynthetic process [GO:0061934] (biological process) Definition: Any process that modulates the frequency, rate or extent of an adenine biosynthetic process. References: PMID:19933844 Relationships: is a type of regulation of purine nucleobase metabolic process [GO:0006141]; is_a GO:0009889; regulates adenine biosynthetic process [GO:0046084]